{
  "gene_symbol": "SLC2A4",
  "gene_name": "Solute carrier family 2, facilitated glucose transporter member 4",
  "term_label": "cellular response to insulin stimulus",
  "gene": "UniProtKB:P14672",
  "term_id": "GO:0032869"
}